{
  "gene_symbol": "RAC3",
  "gene": "UniProtKB:P60763",
  "term_label": "cytoskeleton",
  "gene_name": "Ras-related C3 botulinum toxin substrate 3",
  "term_id": "GO:0005856"
}